{
  "gene_symbol": "SETD5",
  "term_id": "GO:0070210",
  "gene": "UniProtKB:Q9C0A6",
  "gene_name": "Histone-lysine N-methyltransferase SETD5",
  "term_label": "Rpd3L-Expanded complex"
}